{
  "gene": "UniProtKB:Q6T4R5",
  "term_id": "GO:0030154",
  "gene_name": "Actin remodeling regulator NHS",
  "gene_symbol": "NHS",
  "term_label": "cell differentiation"
}